regulation of protein localization to presynapse [GO:1905384] (biological process) Subtypes: negative regulation of protein localization to presynapse [GO:1905385], positive regulation of protein localization to presynapse [GO:1905386] References: PMID:24449494 Sources: GOC:PARL, GOC:TermGenie, GOC:bf, GO_REF:0000058 Relationships: is_a regulation of protein localization to synapse [GO:1902473]; regulates protein localization to presynapse [GO:1905383] Definition: Any process that modulates the frequency, rate or extent of protein localization to presynapse. Also known as: regulation of protein localisation in presynapse, regulation of protein localisation to presynapse, regulation of protein localization in presynapse, regulation of recruitment of presynaptic proteins